{
  "term_label": "ubiquitin-like ligase-substrate adaptor activity",
  "gene_name": "Kelch-like protein 15",
  "term_id": "GO:1990756",
  "gene": "UniProtKB:Q96M94",
  "gene_symbol": "KLHL15"
}